{
  "term_id": "GO:0036503",
  "gene_symbol": "SYVN1",
  "gene_name": "E3 ubiquitin-protein ligase synoviolin",
  "gene": "UniProtKB:Q86TM6",
  "term_label": "ERAD pathway"
}